{
  "gene": "UniProtKB:Q96BK5",
  "term_id": "GO:0010521",
  "gene_symbol": "PINX1",
  "term_label": "telomerase inhibitor activity",
  "gene_name": "PIN2_TERF1-interacting telomerase inhibitor 1"
}